{
  "gene": "UniProtKB:Q9H9P5",
  "gene_symbol": "UNKL",
  "gene_name": "Putative E3 ubiquitin-protein ligase UNKL",
  "term_label": "Unknown molecular function",
  "term_id": "UNKNOWN:0001"
}